long-chain fatty acyl-CoA dehydrogenase activity [GO:0004466] (molecular function) Sources: RHEA:17721 Also known as: long-chain-acyl-CoA dehydrogenase activity, palmitoyl-CoA dehydrogenase activity, palmitoyl-coenzyme A dehydrogenase activity, long-chain acyl-coenzyme A dehydrogenase activity Definition: Catalysis of the reaction: a long-chain 2,3-saturated fatty acyl-CoA + H+ + oxidized [electron-transfer flavoprotein] = a long-chain (2E)-enoyl-CoA + reduced [electron-transfer flavoprotein]. A long-chain fatty acid has an aliphatic tail containing 13 to 22 carbons. Note: While there is not universal consensus on the lengths of short-, medium-, long- and very-long-chain fatty acids, the GO uses the definitions in ChEBI (see CHEBI:26666, CHEBI:59554, CHEBI:15904 and CHEBI:27283). Relationships: is a type of acyl-CoA dehydrogenase activity [GO:0003995]